{
  "gene_name": "Prostaglandin F2-alpha receptor",
  "gene": "UniProtKB:P43088",
  "gene_symbol": "PTGFR",
  "term_label": "inflammatory response",
  "term_id": "GO:0006954"
}